{
  "term_label": "GTPase activity",
  "gene_name": "Ras-related protein Rab-20",
  "gene_symbol": "RAB20",
  "term_id": "GO:0003924",
  "gene": "UniProtKB:Q9NX57"
}